regulation of protein processing in phagocytic vesicle [GO:1903921] (biological process) Relationships: is a type of regulation of protein processing [GO:0070613]; regulates protein processing in phagocytic vesicle [GO:1900756] Definition: Any process that modulates the frequency, rate or extent of protein processing in phagocytic vesicle. Subtypes: negative regulation of protein processing in phagocytic vesicle [GO:1903922], positive regulation of protein processing in phagocytic vesicle [GO:1903923] References: PMID:23325791 Sources: GOC:TermGenie, GOC:als, GO_REF:0000058 Also known as: regulation of protein maturation by peptide bond cleavage in phagocytic vesicle, regulation of protein maturation by peptide bond cleavage in phagosome, regulation of protein maturation by peptide bond hydrolysis in phagocytic vesicle, regulation of protein maturation by peptide bond hydrolysis in phagosome, regulation of protein processing in phagosome, regulation of peptidolysis during protein maturation in phagocytic vesicle, regulation of peptidolysis during protein maturation in phagosome, regulation of protein maturation by proteolysis in phagocytic vesicle, regulation of protein maturation by proteolysis in phagosome